{
  "term_label": "Unknown biological process",
  "term_id": "UNKNOWN:0002",
  "gene_symbol": "TMEM168",
  "gene": "UniProtKB:Q9H0V1",
  "gene_name": "Transmembrane protein 168"
}